{
  "gene_name": "Proton-coupled zinc antiporter SLC30A1",
  "term_label": "membrane",
  "gene": "UniProtKB:Q9Y6M5",
  "term_id": "GO:0016020",
  "gene_symbol": "SLC30A1"
}